{
  "term_label": "membrane",
  "gene": "UniProtKB:O14525",
  "term_id": "GO:0016020",
  "gene_symbol": "ASTN1",
  "gene_name": "Astrotactin-1"
}